methylthiotransferase activity [GO:0035596] (molecular function) Subtypes: tRNA-2-methylthio-N(6)-dimethylallyladenosine(37) synthase activity [GO:0035597], GO:0035598, aspartic acid methylthiotransferase activity [GO:0035599], protein methylthiotransferase activity [GO:0103039] Also known as: MTTase Definition: Catalysis of the addition of a methylthioether group (-SCH3) to a nucleic acid or protein acceptor. Relationships: is a type of alkylthioltransferase activity [GO:0050497] References: PMID:20472640 Sources: GOC:jh2